{
  "gene_symbol": "CHMP6",
  "gene": "UniProtKB:Q96FZ7",
  "term_id": "UNKNOWN:0001",
  "term_label": "Unknown molecular function",
  "gene_name": "Charged multivesicular body protein 6"
}